{
  "term_id": "GO:0000902",
  "gene_name": "Cadherin-19",
  "gene_symbol": "CDH19",
  "term_label": "cell morphogenesis",
  "gene": "UniProtKB:Q9H159"
}